{
  "gene_symbol": "TRPC1",
  "gene_name": "Short transient receptor potential channel 1",
  "term_id": "GO:0070679",
  "term_label": "inositol 1,4,5 trisphosphate binding",
  "gene": "UniProtKB:P48995"
}